{
  "term_label": "SNARE complex",
  "gene_symbol": "SNX4",
  "term_id": "GO:0031201",
  "gene": "UniProtKB:O95219",
  "gene_name": "Sorting nexin-4"
}